{
  "term_label": "thyroid hormone metabolic process",
  "gene_name": "Type II iodothyronine deiodinase",
  "gene_symbol": "DIO2",
  "term_id": "GO:0042403",
  "gene": "UniProtKB:Q92813"
}